{
  "term_id": "GO:0005886",
  "term_label": "plasma membrane",
  "gene_symbol": "HTR3E",
  "gene": "UniProtKB:A5X5Y0",
  "gene_name": "5-hydroxytryptamine receptor 3E"
}